{
  "gene_symbol": "ARB2BP",
  "term_label": "regulatory ncRNA-mediated heterochromatin formation",
  "gene_name": "Putative protein FAM172B",
  "gene": "UniProtKB:A6NC97",
  "term_id": "GO:0031048"
}